{
  "term_label": "negative regulation of transcription by RNA polymerase II",
  "gene_name": "Nuclear receptor corepressor 1",
  "term_id": "GO:0000122",
  "gene_symbol": "NCOR1",
  "gene": "UniProtKB:O75376"
}